tolerance induction dependent upon immune response [GO:0002461] (biological process) Subtypes: tolerance induction to nonself antigen [GO:0002462], peripheral tolerance induction [GO:0002465] Relationships: is a type of adaptive immune response based on somatic recombination of immune receptors built from immunoglobulin superfamily domains [GO:0002460]; is a type of GO:0002507 Regulation: RO_0002211 by regulation of tolerance induction dependent upon immune response [GO:0002652]; negatively regulated by negative regulation of tolerance induction dependent upon immune response [GO:0002653]; positively regulated by positive regulation of tolerance induction dependent upon immune response [GO:0002654] Also known as: immune response-dependent tolerance induction Definition: Tolerance induction dependent upon an immune response, typically a response by a mature T or B cell in the periphery resulting tolerance towards an antigen via induction of anergy, cellular deletion, or regulatory T cell activation. Sources: GOC:jal, GO_REF:0000022, ISBN:0781735149